{
  "term_label": "neuron projection",
  "term_id": "GO:0043005",
  "gene_name": "Acetylcholine receptor subunit delta",
  "gene": "UniProtKB:Q07001",
  "gene_symbol": "CHRND"
}